coumarin 7-hydroxylase activity [GO:0008389] (molecular function) Relationships: is a type of monooxygenase activity [GO:0004497]; is a type of GO:0016705 Also known as: cytochrome P450 CYP2A5 References: PMID:10490589, PMID:2733794 Definition: Catalysis of the reaction: coumarin + O2 + NADPH + H+ = hydroxycoumarin + H2O + NADP+.